{
  "gene_symbol": "RFPL4A",
  "term_label": "regulation of gene expression",
  "gene": "UniProtKB:A6NLU0",
  "gene_name": "Ret finger protein-like 4A",
  "term_id": "GO:0010468"
}